{
  "term_id": "GO:0005549",
  "gene": "UniProtKB:Q8NGR3",
  "gene_name": "Olfactory receptor 1K1",
  "term_label": "odorant binding",
  "gene_symbol": "OR1K1"
}